{
  "gene_symbol": "NAPSA",
  "term_label": "extracellular space",
  "gene": "UniProtKB:O96009",
  "gene_name": "Napsin-A",
  "term_id": "GO:0005615"
}